alphav-beta3 integrin-collagen alpha3(VI) complex [GO:0070464] (cellular component) References: PMID:8387021 Relationships: is a type of plasma membrane protein complex [GO:0098797] Definition: A protein complex that consists of an alphav-beta3 integrin complex bound to the alpha3 chain of type VI collagen; the integrin binds most strongly to unfolded collagen.